{
  "gene_symbol": "UBE2J2",
  "gene": "UniProtKB:Q8N2K1",
  "gene_name": "Ubiquitin-conjugating enzyme E2 J2",
  "term_id": "GO:0000209",
  "term_label": "protein polyubiquitination"
}